metanephric cap morphogenesis [GO:0072186] (biological process) Sources: GOC:mtg_kidney_jan10 Definition: The process in which the anatomical structures of the metanephric cap are generated and organized. The metanephric cap is formed by the condensation of metanephric mesenchymal cells surrounding the ureteric bud tip. Relationships: is a type of metanephric mesenchyme morphogenesis [GO:0072133]; is part of metanephric cap development [GO:0072185]